{
  "gene": "UniProtKB:Q9BYG4",
  "gene_name": "Partitioning defective 6 homolog gamma",
  "term_label": "cell cortex",
  "term_id": "GO:0005938",
  "gene_symbol": "PARD6G"
}